{
  "term_id": "GO:0009966",
  "gene": "UniProtKB:Q14D04",
  "term_label": "regulation of signal transduction",
  "gene_symbol": "VEPH1",
  "gene_name": "Ventricular zone-expressed PH domain-containing protein homolog 1"
}